{
  "gene_symbol": "PYY2",
  "gene": "UniProtKB:Q9NRI6",
  "term_id": "UNKNOWN:0002",
  "gene_name": "Putative peptide YY-2",
  "term_label": "Unknown biological process"
}